head involution [GO:0008258] (biological process) Definition: Movement of the anterior ectoderm to the interior of the embryo. Relationships: is a type of embryonic morphogenesis [GO:0048598]; is part of GO:0001700 Sources: ISBN:0879694238